{
  "gene": "UniProtKB:A6NMZ7",
  "gene_name": "Collagen alpha-6(VI) chain",
  "term_label": "Unknown molecular function",
  "gene_symbol": "COL6A6",
  "term_id": "UNKNOWN:0001"
}